ErbB-3 class receptor binding [GO:0043125] (molecular function) Relationships: is a type of signaling receptor binding [GO:0005102] Also known as: HER3 receptor binding, Neu/ErbB-2 receptor activity Sources: GOC:jl Definition: Binding to the protein-tyrosine kinase receptor ErbB-3/HER3.